methylglyoxal metabolic process [GO:0009438] (biological process) Definition: The chemical reactions and pathways involving methylglyoxal, CH3-CO-CHO, the aldehyde of pyruvic acid. Sources: GOC:ai Also known as: methylglyoxal metabolism, methylglyoxal bypass, methylglyoxal pathway Relationships: is a type of aldehyde metabolic process [GO:0006081]; is a type of ketone metabolic process [GO:0042180] Subtypes: methylglyoxal biosynthetic process [GO:0019242], GO:0036530, methylglyoxal catabolic process [GO:0051596], guanine deglycation, methylglyoxal removal [GO:0106045]